preribosome [GO:0030684] (cellular component) Definition: Any complex of pre-rRNAs, ribosomal proteins, and associated proteins formed during ribosome biogenesis. References: PMID:10567516 Subtypes: GO:0030686, preribosome, large subunit precursor [GO:0030687], preribosome, small subunit precursor [GO:0030688], small-subunit processome [GO:0032040] Relationships: is a type of ribonucleoprotein complex [GO:1990904]